cellular response to glyceraldehyde [GO:1905631] (biological process) References: PMID:11377826 Sources: GOC:TermGenie, GO_REF:0000071 Definition: Any process that results in a change in state or activity of a cell (in terms of movement, secretion, enzyme production, gene expression, etc.) as a result of a glyceraldehyde stimulus. Relationships: is a type of cellular response to monosaccharide stimulus [GO:0071326]; is_a response to glyceraldehyde [GO:1905630]